response to hydroperoxide [GO:0033194] (biological process) Sources: GOC:mah Subtypes: response to lipid hydroperoxide [GO:0006982], response to alkyl hydroperoxide [GO:0033195], cellular response to hydroperoxide [GO:0071447] Definition: Any process that results in a change in state or activity of a cell or an organism (in terms of movement, secretion, enzyme production, gene expression, etc.) as a result of a hydroperoxide stimulus. Hydroperoxides are monosubstitution products of hydrogen peroxide, HOOH. Relationships: is a type of GO:0006979; is a type of response to oxygen-containing compound [GO:1901700]